{
  "gene_name": "Barrier-to-autointegration factor-like protein",
  "gene": "UniProtKB:Q9H503",
  "term_id": "GO:0005634",
  "gene_symbol": "BANF2",
  "term_label": "nucleus"
}